{
  "term_label": "protein K11-linked ubiquitination",
  "gene_name": "Ubiquitin-conjugating enzyme E2 D3",
  "gene": "UniProtKB:P61077",
  "gene_symbol": "UBE2D3",
  "term_id": "GO:0070979"
}